{
  "gene_symbol": "SPANXB1",
  "gene_name": "Sperm protein associated with the nucleus on the X chromosome B1",
  "gene": "UniProtKB:Q9NS25",
  "term_id": "UNKNOWN:0001",
  "term_label": "Unknown molecular function"
}